negative regulation of testicular blood vessel morphogenesis [GO:0061369] (biological process) Also known as: negative regulation of testicular vasculature morphogenesis Relationships: is a type of negative regulation of blood vessel morphogenesis [GO:2000181] Definition: Any process that stops, prevents, or reduces the frequency, rate or extent of blood vessel morphogenesis in the testicle. Sources: GOC:BHF, GOC:dph